outer stripe development [GO:0072058] (biological process) Sources: GOC:mtg_kidney_jan10 Relationships: is a type of anatomical structure development [GO:0048856]; is part of renal outer medulla development [GO:0072054] Definition: The process whose specific outcome is the progression of the outer stripe over time, from its formation to the mature structure. The outer stripe is the region of the kidney outer medulla that lies just below the cortex. The proximal straight tubules (S3) characterize this region.